dendritic cell chemotaxis [GO:0002407] (biological process) Subtypes: myeloid dendritic cell chemotaxis [GO:0002408], GO:0002410 Relationships: is a type of leukocyte chemotaxis [GO:0030595]; is a type of dendritic cell migration [GO:0036336] Definition: The movement of a dendritic cell in response to an external stimulus. References: PMID:15814331, PMID:16056255 Sources: CL:0000451, GOC:add, ISBN:0781735149 Regulation: regulated by regulation of dendritic cell chemotaxis [GO:2000508]; negatively regulated by GO:2000509; positively regulated by positive regulation of dendritic cell chemotaxis [GO:2000510]